{
  "term_id": "GO:0005886",
  "gene_symbol": "CABP1",
  "term_label": "plasma membrane",
  "gene": "UniProtKB:Q9NZU7",
  "gene_name": "Calcium-binding protein 1"
}